folate import across plasma membrane [GO:1904447] (biological process) Relationships: is a type of import across plasma membrane [GO:0098739]; is a type of GO:0098838 References: PMID:19762432 Sources: GOC:BHF, GOC:TermGenie, GOC:hal, GO_REF:0000075 Also known as: folate import into cell, folic acid import across plasma membrane Definition: The directed movement of folic acid from outside of a cell, across the plasma membrane and into the cytosol.